triose-phosphate isomerase activity [GO:0004807] (molecular function) Relationships: is a type of GO:0016861 Sources: RHEA:18585 Also known as: D-glyceraldehyde-3-phosphate aldose-ketose-isomerase activity, D-glyceraldehyde-3-phosphate ketol-isomerase activity, phosphotriose isomerase activity, triose phosphate mutase activity, triose phosphoisomerase activity, triosephosphate isomerase activity, triosephosphate mutase activity Definition: Catalysis of the reaction: D-glyceraldehyde 3-phosphate = dihydroxyacetone phosphate.